{
  "term_label": "cytoplasm",
  "gene_name": "E3 ubiquitin-protein ligase RNF149",
  "gene": "UniProtKB:Q8NC42",
  "gene_symbol": "RNF149",
  "term_id": "GO:0005737"
}